{
  "gene_symbol": "KLK1",
  "term_label": "serine-type endopeptidase activity",
  "gene": "UniProtKB:P06870",
  "gene_name": "Kallikrein-1",
  "term_id": "GO:0004252"
}